chenodeoxycholate 7-alpha-dehydrogenase (NAD+) activity [GO:0106281] (molecular function) References: PMID:12917011 Sources: RHEA:42036 Relationships: is a type of steroid dehydrogenase activity, acting on the CH-OH group of donors, NAD or NADP as acceptor [GO:0033764] Definition: Catalysis of the reaction: chenodeoxycholate + NAD+ = 7-oxolithocholate + H+ + NADH.